{
  "gene": "UniProtKB:Q9Y4F5",
  "gene_symbol": "CEP170B",
  "gene_name": "Centrosomal protein of 170 kDa protein B",
  "term_id": "UNKNOWN:0002",
  "term_label": "Unknown biological process"
}